{
  "gene_name": "Transmembrane protein 272",
  "term_label": "Unknown molecular function",
  "term_id": "UNKNOWN:0001",
  "gene": "UniProtKB:A0A1B0GTI8",
  "gene_symbol": "TMEM272"
}